cellular response to cadmium ion [GO:0071276] (biological process) Sources: GOC:mah Definition: Any process that results in a change in state or activity of a cell (in terms of movement, secretion, enzyme production, gene expression, etc.) as a result of a cadmium (Cd) ion stimulus. Relationships: is a type of response to cadmium ion [GO:0046686]; is a type of cellular response to metal ion [GO:0071248] Also known as: cellular response to cadmium